nucleoside transmembrane transporter activity, against a concentration gradient [GO:0010174] (molecular function) Sources: GOC:tb Also known as: concentrative nucleoside transporter activity Definition: Enables the transfer of a nucleoside, from one side of a membrane to the other, up a concentration gradient. Relationships: is a type of nucleoside transmembrane transporter activity [GO:0005337]; is a type of secondary active transmembrane transporter activity [GO:0015291]